{
  "gene_symbol": "PNMT",
  "gene_name": "Phenylethanolamine N-methyltransferase",
  "term_id": "UNKNOWN:0002",
  "gene": "UniProtKB:P11086",
  "term_label": "Unknown biological process"
}